{
  "gene": "UniProtKB:P33552",
  "term_id": "GO:0019901",
  "gene_name": "Cyclin-dependent kinases regulatory subunit 2",
  "gene_symbol": "CKS2",
  "term_label": "protein kinase binding"
}